cell differentiation in spinal cord [GO:0021515] (biological process) Relationships: is a type of cell differentiation [GO:0030154]; is part of spinal cord development [GO:0021510] References: PMID:11262869 Sources: GOC:cls, GOC:dgh, GOC:dph, GOC:jid, GO_REF:0000021 Definition: The process in which relatively unspecialized cells acquire specialized structural and/or functional features that characterize the cells of the spinal cord. Differentiation includes the processes involved in commitment of a cell to a specific fate. Subtypes: ventral spinal cord interneuron differentiation [GO:0021514], spinal cord motor neuron differentiation [GO:0021522], medial motor column neuron differentiation [GO:0021526], GO:0021527, commissural neuron differentiation in spinal cord [GO:0021528], spinal cord oligodendrocyte cell differentiation [GO:0021529], GO:0021531